{
  "gene": "UniProtKB:A6NK06",
  "term_id": "GO:0005739",
  "gene_name": "Cis-aconitate decarboxylase",
  "term_label": "mitochondrion",
  "gene_symbol": "ACOD1"
}